{
  "term_id": "GO:0003729",
  "term_label": "mRNA binding",
  "gene_name": "Probable ATP-dependent RNA helicase DDX53",
  "gene": "UniProtKB:Q86TM3",
  "gene_symbol": "DDX53"
}